{
  "term_label": "ubiquitin binding",
  "term_id": "GO:0043130",
  "gene_symbol": "PLAA",
  "gene_name": "Phospholipase A-2-activating protein",
  "gene": "UniProtKB:Q9Y263"
}